{
  "gene": "UniProtKB:Q3C1V8",
  "gene_name": "Brain-specific homeobox protein homolog",
  "gene_symbol": "BSX",
  "term_id": "GO:0005634",
  "term_label": "nucleus"
}